{
  "gene": "UniProtKB:Q9HAB8",
  "term_id": "GO:0004632",
  "gene_name": "Phosphopantothenate--cysteine ligase",
  "gene_symbol": "PPCS",
  "term_label": "phosphopantothenate--cysteine ligase activity"
}